{
  "gene": "UniProtKB:Q99929",
  "term_id": "GO:0007423",
  "term_label": "sensory organ development",
  "gene_name": "Achaete-scute homolog 2",
  "gene_symbol": "ASCL2"
}